positive regulation of blood vessel endothelial cell proliferation involved in sprouting angiogenesis [GO:1903589] (biological process) Relationships: is a type of positive regulation of endothelial cell proliferation [GO:0001938]; is a type of regulation of blood vessel endothelial cell proliferation involved in sprouting angiogenesis [GO:1903587]; positively regulates blood vessel endothelial cell proliferation involved in sprouting angiogenesis [GO:0002043] Definition: Any process that activates or increases the frequency, rate or extent of blood vessel endothelial cell proliferation involved in sprouting angiogenesis. Also known as: up regulation of blood vessel endothelial cell proliferation involved in sprouting angiogenesis, up-regulation of blood vessel endothelial cell proliferation involved in sprouting angiogenesis, upregulation of blood vessel endothelial cell proliferation involved in sprouting angiogenesis, activation of blood vessel endothelial cell proliferation involved in sprouting angiogenesis, activation of blood vessel endothelial cell proliferation during sprouting angiogenesis, positive regulation of blood vessel endothelial cell proliferation during sprouting angiogenesis, up regulation of blood vessel endothelial cell proliferation during sprouting angiogenesis, up-regulation of blood vessel endothelial cell proliferation during sprouting angiogenesis, upregulation of blood vessel endothelial cell proliferation during sprouting angiogenesis References: PMID:23388056 Sources: GOC:TermGenie, GO_REF:0000058